{
  "gene": "UniProtKB:O15393",
  "term_id": "GO:0008236",
  "gene_symbol": "TMPRSS2",
  "gene_name": "Transmembrane protease serine 2",
  "term_label": "serine-type peptidase activity"
}